{
  "term_id": "UNKNOWN:0003",
  "gene": "UniProtKB:P0DP71",
  "term_label": "Unknown cellular component",
  "gene_symbol": "FAM236C",
  "gene_name": "Protein FAM236C"
}